{
  "term_id": "UNKNOWN:0003",
  "gene": "UniProtKB:Q96LT6",
  "gene_name": "UPF0739 protein C1orf74",
  "term_label": "Unknown cellular component",
  "gene_symbol": "C1orf74"
}